{
  "term_label": "Unknown biological process",
  "gene": "UniProtKB:Q96D03",
  "gene_name": "DNA damage-inducible transcript 4-like protein",
  "gene_symbol": "DDIT4L",
  "term_id": "UNKNOWN:0002"
}